response to diphenyl ether [GO:1901497] (biological process) Definition: Any process that results in a change in state or activity of a cell or an organism (in terms of movement, secretion, enzyme production, gene expression, etc.) as a result of a diphenyl ether stimulus. Relationships: is a type of GO:0045472 Sources: GOC:TermGenie, GOC:mengo_curators